{
  "gene_name": "C-C chemokine receptor type 6",
  "term_label": "cell chemotaxis",
  "term_id": "GO:0060326",
  "gene": "UniProtKB:P51684",
  "gene_symbol": "CCR6"
}